determination of imaginal disc primordium [GO:0007445] (biological process) Subtypes: determination of genital disc primordium [GO:0035225], determination of wing disc primordium [GO:0035294] Sources: ISBN:0879694238 Relationships: is a type of GO:0045165; is part of imaginal disc development [GO:0007444] Definition: Allocation of embryonic cells to the imaginal disc founder populations, groups of cells that are committed to contribute to the formation of an imaginal disc compartment.